regulation of mitochondrial fusion [GO:0010635] (biological process) Subtypes: GO:0010636, GO:0010637 Relationships: is_a regulation of mitochondrion organization [GO:0010821]; is a type of regulation of anatomical structure morphogenesis [GO:0022603]; regulates mitochondrial fusion [GO:0008053] Definition: Any process that modulates the frequency, rate or extent of merging of two or more mitochondria within a cell to form a single compartment. Sources: GOC:dph, GOC:tb